dol-P-Man:GlcN-acyl-PI alpha-1,4-mannosyltransferase activity [GO:0180041] (molecular function) Relationships: is a type of GPI mannosyltransferase activity [GO:0004376]; is a type of alpha-1,4-mannosyltransferase activity [GO:0051751] Also known as: glycolipid 1,4-alpha-mannosyltransferase activity, GPI-MT-I activity, glycosylphosphatidylinositol-mannosyltransferase I activity Definition: Catalysis of the reaction: a 2-acyl-6-alpha-D-glucosaminyl-1-(1-radyl,2-acyl-sn-glycero-3-phospho)-1D-myo-inositol + a di-trans,poly-cis-dolichyl beta-D-mannosyl phosphate = a 2-acyl-6-(alpha-D-mannosyl-(1->4)-alpha-D-glucosaminyl)-1-(1-radyl,2-acyl-sn-glycero-3-phospho)-1D-myo-inositol + a di-trans,poly-cis-dolichyl phosphate + H+. References: PMID:11226175, PMID:15635094 Sources: RHEA:60500